{
  "gene_symbol": "HPS6",
  "gene": "UniProtKB:Q86YV9",
  "gene_name": "BLOC-2 complex member HPS6",
  "term_id": "GO:0072657",
  "term_label": "protein localization to membrane"
}